1-phosphatidyl-1D-myo-inositol 3,5-bisphosphate metabolic process [GO:1903100] (biological process) References: PMID:19037259 Sources: GOC:TermGenie, GOC:bhm, GO_REF:0000068 Definition: The chemical reactions and pathways involving 1-phosphatidyl-1D-myo-inositol 3,5-bisphosphate. Relationships: is a type of phosphatidylinositol metabolic process [GO:0046488] Also known as: 1-phosphatidyl-1D-myo-inositol 3,5-bisphosphate metabolism Subtypes: 1-phosphatidyl-1D-myo-inositol 3,5-bisphosphate catabolic process [GO:1903101], 1-phosphatidyl-1D-myo-inositol 3,5-bisphosphate biosynthetic process [GO:1903102]